estrogen 2-hydroxylase activity [GO:0101021] (molecular function) Definition: Catalysis of the reaction: estrogen + reduced [NADPH--hemoprotein reductase] + O2 = 2-hydroxyestrogen + H+ + H2O + oxidized [NADPH--hemoprotein reductase]. Also known as: oestrogen 2-hydroxylase activity Relationships: is a type of steroid hydroxylase activity [GO:0008395]; is a type of oxidoreductase activity, acting on paired donors, with incorporation or reduction of molecular oxygen, reduced flavin or flavoprotein as one donor, and incorporation of one atom of oxygen [GO:0016712] References: PMID:14559847 Sources: GOC:BHF, GOC:rl